glycosylation-dependent protein binding [GO:0140032] (molecular function) Relationships: is a type of modification-dependent protein binding [GO:0140030] Definition: Binding to a protein upon glycosylation of the target protein. Note: This term should only be used when the binding is shown to require glycosylation of the target protein: the interaction needs to be tested with and without the PTM. The binding does not need to be at the site of glycosylation. It may be that the glycosylation causes a conformational change that allows binding of the protein to another region; this type of glycosylation-dependent protein binding is valid for annotation to this term. References: PMID:26060076